{
  "term_label": "regulation of response to osmotic stress",
  "gene": "UniProtKB:Q15049",
  "gene_symbol": "MLC1",
  "term_id": "GO:0047484",
  "gene_name": "Membrane protein MLC1"
}